{
  "term_id": "GO:0000978",
  "term_label": "RNA polymerase II cis-regulatory region sequence-specific DNA binding",
  "gene": "UniProtKB:Q9Y6R6",
  "gene_name": "Zinc finger protein 780B",
  "gene_symbol": "ZNF780B"
}